protein polyufmylation [GO:1990564] (biological process) Relationships: is a type of protein ufmylation [GO:0071569] Subtypes: protein K69-linked ufmylation [GO:1990592] Definition: Covalent attachment of the ubiquitin-like protein UFM1 to a protein, forming an UFM1 chain. References: PMID:25219498